immunoglobulin receptor binding [GO:0034987] (molecular function) Definition: Binding to one or more specific sites on an immunoglobulin receptor molecule. Relationships: is a type of signaling receptor binding [GO:0005102] Also known as: Fc receptor binding Sources: GOC:BHF, GOC:vk Subtypes: Fc-gamma receptor I complex binding [GO:0034988]